{
  "gene_symbol": "ASPA",
  "term_id": "GO:0016811",
  "term_label": "hydrolase activity, acting on carbon-nitrogen (but not peptide) bonds, in linear amides",
  "gene_name": "Aspartoacylase",
  "gene": "UniProtKB:P45381"
}